{
  "gene_name": "Ubiquitin-like protein ATG12",
  "term_label": "autophagosome assembly",
  "gene": "UniProtKB:O94817",
  "term_id": "GO:0000045",
  "gene_symbol": "ATG12"
}